cobalt-precorrin-7 C15-methyltransferase activity [GO:0043777] (molecular function) Definition: Catalysis of the reaction: cobalt-precorrin 7 + S-adenosyl-L-methionine = cobalt-precorrin 8 + S-adenosyl-L-homocysteine + CO2. Relationships: is a type of GO:0008168 Also known as: precorrin-6 methyltransferase, precorrin-6Y C5,15-methyltransferase (decarboxylating), precorrin-6Y methylase, cobalt-precorrin 7 C15-methyltransferase activity Sources: MetaCyc:RXN-8767